{
  "gene": "UniProtKB:Q8WVC0",
  "gene_name": "RNA polymerase-associated protein LEO1",
  "term_label": "nucleus",
  "term_id": "GO:0005634",
  "gene_symbol": "LEO1"
}